{
  "gene_symbol": "MTCP1",
  "gene_name": "Protein p13 MTCP-1",
  "term_id": "GO:0043539",
  "gene": "UniProtKB:P56278",
  "term_label": "protein serine/threonine kinase activator activity"
}